auxin conjugate metabolic process [GO:0010249] (biological process) Sources: GOC:sm Relationships: is a type of GO:0009850 Definition: The chemical reactions and pathways involving auxin conjugates, a bound form of auxin. Also known as: auxin conjugate metabolism